{
  "gene": "UniProtKB:Q9UMZ2",
  "term_label": "clathrin coat of trans-Golgi network vesicle",
  "gene_symbol": "SYNRG",
  "gene_name": "Synergin gamma",
  "term_id": "GO:0030130"
}